negative regulation of synaptic assembly at neuromuscular junction [GO:0045886] (biological process) Sources: GOC:go_curators Definition: Any process that stops, prevents, or reduces the frequency, rate or extent of synaptic assembly at neuromuscular junction. Relationships: is a type of regulation of synaptic assembly at neuromuscular junction [GO:0008582]; is a type of GO:0048640; is a type of negative regulation of synapse assembly [GO:0051964]; is a type of negative regulation of neuromuscular junction development [GO:1904397]; negatively regulates GO:0051124 Also known as: down regulation of synaptic growth at neuromuscular junction, down-regulation of synaptic growth at neuromuscular junction, downregulation of synaptic growth at neuromuscular junction, inhibition of synaptic growth at neuromuscular junction, negative regulation of synaptic growth at neuromuscular junction